{
  "term_label": "microtubule cytoskeleton",
  "gene_symbol": "MAST3",
  "term_id": "GO:0015630",
  "gene": "UniProtKB:O60307",
  "gene_name": "Microtubule-associated serine_threonine-protein kinase 3"
}